{
  "gene": "UniProtKB:O43261",
  "gene_name": "Leukemia-associated protein 1",
  "gene_symbol": "DLEU1",
  "term_label": "Unknown biological process",
  "term_id": "UNKNOWN:0002"
}